positive regulation of intestinal epithelial structure maintenance [GO:0060731] (biological process) Definition: Any process the increases the rate, frequency or extent of intestinal epithelial structure maintenance, a tissue homeostatic process required for the maintenance of the structure of the intestinal epithelium. Sources: GOC:dph, GOC:tb Relationships: is a type of positive regulation of digestive system process [GO:0060456]; is a type of regulation of intestinal epithelial structure maintenance [GO:0060730]; positively regulates intestinal epithelial structure maintenance [GO:0060729]